{
  "gene_name": "Proto-oncogene vav",
  "term_id": "GO:0016477",
  "term_label": "cell migration",
  "gene_symbol": "VAV1",
  "gene": "UniProtKB:P15498"
}